{
  "term_label": "organic acid metabolic process",
  "term_id": "GO:0006082",
  "gene": "UniProtKB:Q7Z449",
  "gene_name": "Cytochrome P450 2U1",
  "gene_symbol": "CYP2U1"
}